{
  "gene": "UniProtKB:Q9Y581",
  "gene_symbol": "INSL6",
  "term_label": "Unknown molecular function",
  "term_id": "UNKNOWN:0001",
  "gene_name": "Insulin-like peptide INSL6"
}